{
  "term_id": "GO:0000981",
  "gene_symbol": "HOXA5",
  "term_label": "DNA-binding transcription factor activity, RNA polymerase II-specific",
  "gene_name": "Homeobox protein Hox-A5",
  "gene": "UniProtKB:P20719"
}